{
  "gene_symbol": "NPAT",
  "term_id": "GO:0003712",
  "term_label": "transcription coregulator activity",
  "gene": "UniProtKB:Q14207",
  "gene_name": "Protein NPAT"
}